CDP metabolic process [GO:0046704] (BP) Subtypes: CDP biosynthetic process [GO:0046705], CDP catabolic process [GO:0046706] Relationships: is a type of GO:0009193; is a type of pyrimidine ribonucleotide metabolic process [GO:0009218] Definition: The chemical reactions and pathways involving CDP, cytidine (5'-)diphosphate. Also known as: CDP metabolism Sources: GOC:ai